{
  "gene_symbol": "ZHX1-C8orf76",
  "term_id": "UNKNOWN:0003",
  "term_label": "Unknown cellular component",
  "gene": "UniProtKB:Q96EF9",
  "gene_name": "Zinc fingers and homeoboxes protein 1, isoform 2"
}